{
  "gene": "UniProtKB:Q5T764",
  "gene_symbol": "IFIT1B",
  "gene_name": "Interferon-induced protein with tetratricopeptide repeats 1B",
  "term_id": "GO:0005829",
  "term_label": "cytosol"
}